{
  "gene": "UniProtKB:O95007",
  "gene_name": "Olfactory receptor 6B1",
  "term_label": "plasma membrane",
  "term_id": "GO:0005886",
  "gene_symbol": "OR6B1"
}